{
  "term_label": "Unknown molecular function",
  "gene_symbol": "PDHB",
  "term_id": "UNKNOWN:0001",
  "gene": "UniProtKB:P11177",
  "gene_name": "Pyruvate dehydrogenase E1 component subunit beta, mitochondrial"
}